{
  "term_id": "GO:0045087",
  "gene_symbol": "TRIM62",
  "term_label": "innate immune response",
  "gene": "UniProtKB:Q9BVG3",
  "gene_name": "E3 ubiquitin-protein ligase TRIM62"
}